{
  "gene_symbol": "MT1A",
  "term_label": "detoxification of copper ion",
  "term_id": "GO:0010273",
  "gene": "UniProtKB:P04731",
  "gene_name": "Metallothionein-1A"
}